interferon regulatory factor 7 complex [GO:0097074] (cellular component) Relationships: is a type of interferon regulatory factor complex [GO:0097071] References: PMID:18068231 Sources: GOC:cna Definition: An interferon regulatory factor complex that consists of a homodimer of interferon regulatory factor 7. Also known as: IRF7:IRF7 complex